{
  "term_label": "CoA-ligase activity",
  "term_id": "GO:0016405",
  "gene": "UniProtKB:Q4G176",
  "gene_name": "Malonate--CoA ligase ACSF3, mitochondrial",
  "gene_symbol": "ACSF3"
}